{
  "gene_symbol": "UACA",
  "term_label": "negative regulation of inflammatory response",
  "gene": "UniProtKB:Q9BZF9",
  "gene_name": "Uveal autoantigen with coiled-coil domains and ankyrin repeats",
  "term_id": "GO:0050728"
}